{
  "term_label": "Unknown molecular function",
  "gene_name": "Nucleolar complex protein 4 homolog",
  "gene_symbol": "NOC4L",
  "gene": "UniProtKB:Q9BVI4",
  "term_id": "UNKNOWN:0001"
}